{
  "gene_name": "Keratin-associated protein 1-4",
  "gene": "UniProtKB:P0C5Y4",
  "term_id": "UNKNOWN:0003",
  "term_label": "Unknown cellular component",
  "gene_symbol": "KRTAP1-4"
}